{
  "gene_symbol": "SIGLEC1",
  "term_label": "late endosome",
  "term_id": "GO:0005770",
  "gene": "UniProtKB:Q9BZZ2",
  "gene_name": "Sialoadhesin"
}